{
  "gene_symbol": "TMUB1",
  "term_label": "ERAD pathway",
  "gene_name": "Transmembrane and ubiquitin-like domain-containing protein 1",
  "gene": "UniProtKB:Q9BVT8",
  "term_id": "GO:0036503"
}